{
  "term_label": "Unknown biological process",
  "term_id": "UNKNOWN:0002",
  "gene": "UniProtKB:Q6ZUA9",
  "gene_symbol": "MROH5",
  "gene_name": "Maestro heat-like repeat family member 5"
}